{
  "term_label": "sulfur dioxygenase activity",
  "gene": "UniProtKB:O95571",
  "gene_name": "Persulfide dioxygenase ETHE1, mitochondrial",
  "term_id": "GO:0050313",
  "gene_symbol": "ETHE1"
}